hypophysis morphogenesis [GO:0048850] (biological process) Definition: The process in which the anatomical structures of the hypophysis are generated and organized. The pituitary gland is an endocrine gland that secretes hormones that regulate many other glands. Relationships: is a type of GO:0022612; BFO_0000050 pituitary gland development [GO:0021983]; is part of GO:0048852 Sources: GOC:cls, GOC:dgh, GOC:dph, GOC:jid Also known as: pituitary gland morphogenesis